{
  "term_label": "neuron projection",
  "gene": "UniProtKB:P23219",
  "gene_symbol": "PTGS1",
  "term_id": "GO:0043005",
  "gene_name": "Prostaglandin G_H synthase 1"
}